{
  "term_id": "GO:0098632",
  "gene_name": "Leucine-rich repeat-containing protein 4B",
  "gene_symbol": "LRRC4B",
  "term_label": "cell-cell adhesion mediator activity",
  "gene": "UniProtKB:Q9NT99"
}